response to oxidopamine [GO:1905841] (biological process) Relationships: is a type of response to catecholamine [GO:0071869] Definition: Any process that results in a change in state or activity of a cell or an organism (in terms of movement, secretion, enzyme production, gene expression, etc.) as a result of an oxidopamine stimulus. Subtypes: cellular response to oxidopamine [GO:1905842] References: PMID:23721876 Sources: GOC:TermGenie, GOC:rz, GO_REF:0000071